positive regulation of telium development [GO:0075277] (biological process) Relationships: is a type of GO:0075261; is a type of GO:0075276; positively regulates telium development [GO:0075275] Sources: GOC:pamgo_curators Definition: Any process that activates, maintains or increases the frequency, rate or extent of telium development, a process that leads to the formation of a teliospore-bearing sorus of the rust fungi.